{
  "term_id": "GO:0006637",
  "gene": "UniProtKB:Q9Y305",
  "term_label": "acyl-CoA metabolic process",
  "gene_symbol": "ACOT9",
  "gene_name": "Acyl-coenzyme A thioesterase 9, mitochondrial"
}